{
  "gene": "UniProtKB:O75964",
  "term_label": "proton motive force-driven ATP synthesis",
  "gene_symbol": "ATP5MG",
  "term_id": "GO:0015986",
  "gene_name": "ATP synthase subunit g, mitochondrial"
}